{
  "gene_name": "Spatacsin",
  "term_id": "GO:0048489",
  "gene_symbol": "SPG11",
  "gene": "UniProtKB:Q96JI7",
  "term_label": "synaptic vesicle transport"
}